{
  "gene_symbol": "CCDC122",
  "gene_name": "Coiled-coil domain-containing protein 122",
  "gene": "UniProtKB:Q5T0U0",
  "term_label": "Unknown biological process",
  "term_id": "UNKNOWN:0002"
}